site of double-strand break [GO:0035861] (cellular component) Also known as: site of DSB, DNA damage foci, DNA damage focus, IRIF, ionizing radiation-induced foci References: PMID:20096808, PMID:21035408 Sources: GOC:bf, GOC:mah, GOC:vw Relationships: is a type of site of DNA damage [GO:0090734] Definition: A region of a chromosome at which a DNA double-strand break has occurred. DNA damage signaling and repair proteins accumulate at the lesion to respond to the damage and repair the DNA to form a continuous DNA helix.